{
  "term_label": "Unknown molecular function",
  "gene_name": "Plexin domain-containing protein 1",
  "gene": "UniProtKB:Q8IUK5",
  "gene_symbol": "PLXDC1",
  "term_id": "UNKNOWN:0001"
}